{
  "gene_name": "Interleukin-1 receptor-like 1",
  "term_id": "GO:0038172",
  "term_label": "interleukin-33-mediated signaling pathway",
  "gene": "UniProtKB:Q01638",
  "gene_symbol": "IL1RL1"
}